G-protein alpha(i)1-synembrin complex [GO:0071154] (cellular component) Relationships: is a type of GO:0140535 Also known as: Ric-8A G(i) alpha-1 subunit complex, Ric-8A G(i) alpha-2 subunit complex References: PMID:12509430 Sources: GOC:mah Definition: A protein complex formed by the association of the guanine nucleotide exchange factor synembrin with the alpha(i)1 subunit of a heterotrimeric G protein.